negative regulation of coagulation [GO:0050819] (biological process) Definition: Any process that stops, prevents, or reduces the frequency, rate or extent of coagulation. Sources: GOC:ai Also known as: down regulation of coagulation, down-regulation of coagulation, downregulation of coagulation, negative regulation of clotting, inhibition of coagulation, anticoagulant activity Relationships: is a type of regulation of coagulation [GO:0050818]; is a type of negative regulation of multicellular organismal process [GO:0051241]; negatively regulates coagulation [GO:0050817] Subtypes: negative regulation of blood coagulation [GO:0030195]